{
  "term_id": "GO:0006325",
  "gene_name": "GATA zinc finger domain-containing protein 1",
  "gene": "UniProtKB:Q8WUU5",
  "gene_symbol": "GATAD1",
  "term_label": "chromatin organization"
}